{
  "term_id": "GO:0001788",
  "gene_symbol": "FCGR2C",
  "gene_name": "Low affinity immunoglobulin gamma Fc region receptor II-c",
  "term_label": "antibody-dependent cellular cytotoxicity",
  "gene": "UniProtKB:P31995"
}